telomerase RNA localization [GO:0090672] (BP) Subtypes: telomerase RNA localization to Cajal body [GO:0090671] Definition: Any process in which telomerase RNA is transported to, or maintained in, a specific location. Relationships: is a type of RNA localization [GO:0006403] References: PMID:25467444 Sources: GOC:BHF, GOC:BHF_telomere, GOC:nc